{
  "gene_name": "C-type lectin domain family 4 member G",
  "term_id": "GO:0038187",
  "gene": "UniProtKB:Q6UXB4",
  "term_label": "pattern recognition receptor activity",
  "gene_symbol": "CLEC4G"
}